negative regulation of lymphocyte migration [GO:2000402] (biological process) Subtypes: negative regulation of lymphocyte chemotaxis [GO:1901624], negative regulation of T cell migration [GO:2000405] Definition: Any process that stops, prevents or reduces the frequency, rate or extent of lymphocyte migration. Sources: GOC:mah Relationships: is a type of negative regulation of mononuclear cell migration [GO:0071676]; is a type of regulation of lymphocyte migration [GO:2000401]; negatively regulates GO:0072676